{
  "gene_name": "FHF complex subunit HOOK-interacting protein 1B",
  "gene_symbol": "FHIP1B",
  "term_id": "GO:0007032",
  "gene": "UniProtKB:Q8N612",
  "term_label": "endosome organization"
}